calcium ion regulated lysosome exocytosis [GO:1990927] (biological process) Relationships: is a type of calcium-ion regulated exocytosis [GO:0017156] References: PMID:10725327, PMID:11511344 Definition: The process of secretion by a cell that results in the release of intracellular molecules contained within a lysosome by fusion of the vesicle with the plasma membrane of a cell, induced by a rise in cytosolic calcium-ion levels.